{
  "gene_name": "Protein transport protein Sec61 subunit alpha isoform 1",
  "gene": "UniProtKB:P61619",
  "gene_symbol": "SEC61A1",
  "term_label": "post-translational protein targeting to membrane, translocation",
  "term_id": "GO:0031204"
}